{
  "gene_name": "Midasin",
  "gene": "UniProtKB:Q9NU22",
  "term_id": "GO:0005634",
  "gene_symbol": "MDN1",
  "term_label": "nucleus"
}